{
  "gene": "UniProtKB:Q15050",
  "term_id": "GO:0000447",
  "gene_symbol": "RRS1",
  "gene_name": "Ribosome biogenesis regulatory protein homolog",
  "term_label": "endonucleolytic cleavage in ITS1 to separate SSU-rRNA from 5.8S rRNA and LSU-rRNA from tricistronic rRNA transcript (SSU-rRNA, 5.8S rRNA, LSU-rRNA)"
}